{
  "term_label": "Unknown biological process",
  "gene_symbol": "TMEM184C",
  "term_id": "UNKNOWN:0002",
  "gene": "UniProtKB:Q9NVA4",
  "gene_name": "Transmembrane protein 184C"
}